{
  "term_id": "UNKNOWN:0001",
  "gene_name": "Single-pass membrane and coiled-coil domain-containing protein 3",
  "gene_symbol": "SMCO3",
  "gene": "UniProtKB:A2RU48",
  "term_label": "Unknown molecular function"
}